bilirubin transport [GO:0015723] (biological process) Definition: The directed movement of bilirubin into, out of or within a cell, or between cells, by means of some agent such as a transporter or pore. Sources: GOC:krc Relationships: is a type of dicarboxylic acid transport [GO:0006835]; is a type of GO:0071705